{
  "gene": "UniProtKB:Q9H5N1",
  "gene_name": "Rab GTPase-binding effector protein 2",
  "term_id": "UNKNOWN:0002",
  "term_label": "Unknown biological process",
  "gene_symbol": "RABEP2"
}